meiotic interphase [GO:0051328] (BP) Subtypes: meiotic interphase II [GO:0044844] Note: Note that this term should not be used for direct annotation. If you are trying to make an annotation to x phase, it is likely that the correct annotation is 'regulation of x/y phase transition' or to a process which occurs during the reported phase (i.e mitotic DNA replication for mitotic S-phase). To capture the phase when a specific location or process is observed, the phase term can be used in an annotation extension (PMID:24885854) applied to a cellular component term (with the relation exists_during) or a biological process term (with the relation happens_during). Sources: GOC:mtg_cell_cycle Relationships: is_a interphase [GO:0051325]; is a type of meiotic cell cycle phase [GO:0098762] Also known as: interphase of meiotic cell cycle Definition: The cell cycle phase which begins after cytokinesis and ends when meiotic prophase begins. Meiotic cells have an interphase after each meiotic division, but only interphase I involves replication of the cell's DNA.